{
  "gene_symbol": "IGHV3OR16-12",
  "term_label": "antigen binding",
  "gene_name": "Immunoglobulin heavy variable 3_OR16-12 (non-functional) (Fragment)",
  "gene": "UniProtKB:A0A075B7B8",
  "term_id": "GO:0003823"
}